{
  "gene": "UniProtKB:Q9BSG5",
  "gene_name": "Retbindin",
  "gene_symbol": "RTBDN",
  "term_id": "GO:0032217",
  "term_label": "riboflavin transmembrane transporter activity"
}